dorsal closure, elongation of leading edge cells [GO:0007394] (biological process) Definition: The change in shape of cells at the dorsal-most (leading) edge of the epidermis from being polygonal to being elongated in the dorsal/ventral axis. References: PMID:12147138 Relationships: is_a GO:0009826; is a type of regulation of embryonic cell shape [GO:0016476]; is a type of embryonic morphogenesis [GO:0048598]; BFO_0000050 GO:0007392